zinc D-Ala-D-Ala carboxypeptidase activity [GO:0009046] (molecular function) Definition: Catalysis of the cleavage of the D-alanyl-D-alanine bond in (Ac)2-L-lysyl-D-alanyl-D-alanine. Sources: EC:3.4.17.14 Also known as: DD-carboxypeptidase, D-alanyl-D-alanine hydrolase activity, D-alanyl-D-alanine-cleaving carboxypeptidase activity, DD-carboxypeptidase-transpeptidase activity, G enzyme, Zn(2+) G peptidase activity, Zn2+ G peptidase activity Relationships: is a type of metallocarboxypeptidase activity [GO:0004181]